{
  "term_id": "GO:0005246",
  "gene": "UniProtKB:Q06432",
  "gene_name": "Voltage-dependent calcium channel gamma-1 subunit",
  "term_label": "calcium channel regulator activity",
  "gene_symbol": "CACNG1"
}